{
  "term_label": "nucleolus",
  "gene_symbol": "ADAR",
  "gene_name": "Double-stranded RNA-specific adenosine deaminase",
  "term_id": "GO:0005730",
  "gene": "UniProtKB:P55265"
}